{
  "term_id": "GO:0003735",
  "gene_symbol": "RPL15",
  "gene": "UniProtKB:P61313",
  "term_label": "structural constituent of ribosome",
  "gene_name": "Large ribosomal subunit protein eL15"
}